{
  "gene_symbol": "THRB",
  "gene": "UniProtKB:P10828",
  "gene_name": "Thyroid hormone receptor beta",
  "term_id": "GO:0030154",
  "term_label": "cell differentiation"
}